{
  "gene_symbol": "GUCY2D",
  "gene": "UniProtKB:Q02846",
  "gene_name": "Retinal guanylyl cyclase 1",
  "term_label": "receptor guanylyl cyclase signaling pathway",
  "term_id": "GO:0007168"
}